{
  "term_id": "UNKNOWN:0003",
  "term_label": "Unknown cellular component",
  "gene": "UniProtKB:Q96BA8",
  "gene_symbol": "CREB3L1",
  "gene_name": "Cyclic AMP-responsive element-binding protein 3-like protein 1"
}